fruit development [GO:0010154] (biological process) Relationships: is_a reproductive structure development [GO:0048608] Sources: GOC:sm Definition: The process whose specific outcome is the progression of the fruit over time, from its formation to the mature structure. The fruit is a reproductive body of a seed plant.